kinesis [GO:0042465] (biological process) Sources: GOC:jl, ISBN:0192801023 Relationships: is a type of GO:0009605 Definition: The movement of a cell or organism in response to a stimulus in which the rate of movement depends on the intensity (rather than the direction) of the stimulus. Subtypes: GO:0042466, orthokinesis [GO:0042467], klinokinesis [GO:0042468]